regulation of spindle checkpoint [GO:0090231] (biological process) Subtypes: positive regulation of spindle checkpoint [GO:0090232], negative regulation of spindle checkpoint [GO:0090233], GO:1903504, regulation of meiosis I spindle assembly checkpoint [GO:1905325] Definition: Any process that modulates the rate, frequency, or extent of the spindle checkpoint, a cell cycle checkpoint that delays the metaphase/anaphase transition until the spindle is correctly assembled and oriented, and chromosomes are attached to the spindle. Sources: GOC:ascb_2009, GOC:dph, GOC:tb Note: Note that this term should not be used for direct manual annotation as it should always be possible to specify the type of checkpoint (i.e mitotic spindle or DNA damage etc). Relationships: is a type of GO:1901976; regulates spindle checkpoint signaling [GO:0031577]